{
  "term_label": "SAM complex",
  "term_id": "GO:0001401",
  "gene": "UniProtKB:Q13505",
  "gene_name": "Metaxin-1",
  "gene_symbol": "MTX1"
}